{
  "gene_symbol": "MLLT10",
  "term_id": "GO:0006357",
  "term_label": "regulation of transcription by RNA polymerase II",
  "gene_name": "Protein AF-10",
  "gene": "UniProtKB:P55197"
}